{
  "gene": "UniProtKB:Q9Y4A9",
  "gene_name": "Olfactory receptor 10H1",
  "gene_symbol": "OR10H1",
  "term_label": "detection of chemical stimulus involved in sensory perception of smell",
  "term_id": "GO:0050911"
}